atrazine chlorohydrolase activity [GO:0018788] (molecular function) Also known as: AtzA Definition: Catalysis of the reaction: atrazine + H2O = chloride + H+ + hydroxyatrazine. Sources: RHEA:11312 Relationships: is a type of hydrolase activity, acting on acid halide bonds, in C-halide compounds [GO:0019120]